{
  "gene_symbol": "KLC4",
  "term_label": "kinesin binding",
  "gene": "UniProtKB:Q9NSK0",
  "gene_name": "Kinesin light chain 4",
  "term_id": "GO:0019894"
}